{
  "gene": "UniProtKB:O60729",
  "term_id": "GO:0005730",
  "gene_name": "Dual specificity protein phosphatase CDC14B",
  "gene_symbol": "CDC14B",
  "term_label": "nucleolus"
}